{
  "gene": "UniProtKB:Q5JT25",
  "term_label": "intracellular protein transport",
  "gene_name": "Ras-related protein Rab-41",
  "term_id": "GO:0006886",
  "gene_symbol": "RAB41"
}